{
  "gene_name": "Olfactory receptor 6C4",
  "term_id": "GO:0005886",
  "term_label": "plasma membrane",
  "gene": "UniProtKB:Q8NGE1",
  "gene_symbol": "OR6C4"
}